{
  "gene": "UniProtKB:O75934",
  "term_id": "UNKNOWN:0002",
  "gene_name": "Pre-mRNA-splicing factor SPF27",
  "gene_symbol": "BCAS2",
  "term_label": "Unknown biological process"
}